{
  "gene": "UniProtKB:Q6ZP80",
  "term_label": "Unknown biological process",
  "term_id": "UNKNOWN:0002",
  "gene_name": "Transmembrane protein 182",
  "gene_symbol": "TMEM182"
}